lumenal side of trans-Golgi cisternae membrane [GO:0160289] (cellular component) Definition: The membrane leaflet of the trans-Golgi cisternae membrane that faces the Golgi lumen. It is involved in the final steps of glycan processing, proteolytic modification, and cargo maturation prior to sorting at the trans-Golgi network. References: PMID:34597626, PMID:38307322, PMID:6121819 Also known as: lumenal face of trans-Golgi cisternae membrane, lumenal leaflet of trans-Golgi cisternae membrane, lumenal side of Golgi trans cisternae membrane Relationships: is a type of lumenal side of membrane [GO:0098576]; is part of GO:1990676